negative regulation of L-lysine import across plasma membrane [GO:1905009] (biological process) Also known as: negative regulation of lysine import, down regulation of L-lysine import into cell, down-regulation of L-lysine import into cell, downregulation of L-lysine import into cell, negative regulation of L-lysine import into cell, negative regulation of lysine uptake, inhibition of L-lysine import into cell Definition: Any process that stops, prevents or reduces the frequency, rate or extent of L-lysine import into cell. Relationships: is_a GO:0032891; is a type of GO:0034763; is a type of negative regulation of amino acid transport [GO:0051956]; is a type of regulation of L-lysine import across plasma membrane [GO:1905008]; negatively regulates L-lysine import across plasma membrane [GO:0097639] References: PMID:7499219 Sources: GOC:TermGenie, GO_REF:0000058